{
  "gene": "UniProtKB:Q9HB29",
  "gene_name": "Interleukin-1 receptor-like 2",
  "term_id": "GO:0005886",
  "term_label": "plasma membrane",
  "gene_symbol": "IL1RL2"
}